{
  "gene_symbol": "HMHB1",
  "term_label": "Unknown biological process",
  "term_id": "UNKNOWN:0002",
  "gene_name": "Minor histocompatibility protein HB-1",
  "gene": "UniProtKB:O97980"
}